{
  "gene_name": "Motile sperm domain-containing protein 2",
  "term_label": "endomembrane system",
  "gene": "UniProtKB:Q8NHP6",
  "gene_symbol": "MOSPD2",
  "term_id": "GO:0012505"
}